{
  "gene_name": "Keratin, type II cytoskeletal 4",
  "term_label": "intermediate filament organization",
  "gene": "UniProtKB:P19013",
  "gene_symbol": "KRT4",
  "term_id": "GO:0045109"
}